{
  "gene": "UniProtKB:Q9HAC8",
  "term_label": "Unknown biological process",
  "gene_symbol": "UBTD1",
  "gene_name": "Ubiquitin domain-containing protein 1",
  "term_id": "UNKNOWN:0002"
}